{
  "gene_symbol": "CHRDL2",
  "gene": "UniProtKB:Q6WN34",
  "term_id": "GO:0036122",
  "gene_name": "Chordin-like protein 2",
  "term_label": "BMP binding"
}